{
  "term_id": "GO:0030514",
  "gene_symbol": "SKOR2",
  "term_label": "negative regulation of BMP signaling pathway",
  "gene": "UniProtKB:Q2VWA4",
  "gene_name": "SKI family transcriptional corepressor 2"
}